{
  "gene": "UniProtKB:Q9ULB5",
  "gene_name": "Cadherin-7",
  "term_label": "cell morphogenesis",
  "term_id": "GO:0000902",
  "gene_symbol": "CDH7"
}